{
  "gene": "UniProtKB:Q7Z2V1",
  "gene_symbol": "C16orf82",
  "term_label": "Unknown molecular function",
  "gene_name": "Protein TNT",
  "term_id": "UNKNOWN:0001"
}